sensory perception of touch [GO:0050975] (biological process) Definition: The series of events required for an organism to receive a touch stimulus, convert it to a molecular signal, and recognize and characterize the signal. This is a neurological process. The perception of touch in animals is mediated by mechanoreceptors in the skin and mucous membranes and is the sense by which contact with objects gives evidence as to certain of their qualities. Different types of touch can be perceived (for example, light, coarse, pressure and tickling) and the stimulus may be external or internal (e.g. the feeling of a full stomach). Also known as: perception of touch, tactile sense, taction, tactition Relationships: is a type of sensory perception of mechanical stimulus [GO:0050954] Sources: GOC:ai